{
  "gene_symbol": "KRT73",
  "gene": "UniProtKB:Q86Y46",
  "term_label": "keratin filament",
  "gene_name": "Keratin, type II cytoskeletal 73",
  "term_id": "GO:0045095"
}